detection of unfolded protein [GO:0002235] (BP) Relationships: is a type of GO:0006986; is_a detection of chemical stimulus [GO:0009593] Definition: The series of events in which an unfolded protein stimulus is received and converted into a molecular signal. References: PMID:15226511, PMID:7765470 Sources: GOC:add